{
  "term_label": "plasma membrane",
  "gene_name": "NALCN channel auxiliary factor 1",
  "term_id": "GO:0005886",
  "gene_symbol": "NALF1",
  "gene": "UniProtKB:B1AL88"
}